{
  "gene_symbol": "CHST7",
  "gene": "UniProtKB:Q9NS84",
  "term_id": "GO:0008459",
  "term_label": "chondroitin 6-sulfotransferase activity",
  "gene_name": "Carbohydrate sulfotransferase 7"
}